regulation of cellular response to phosphate starvation [GO:0140255] (biological process) Subtypes: positive regulation of cellular response to phosphate starvation [GO:0080040], GO:0140256 References: PMID:29414789 Definition: Any process that modulates the frequency, rate or extent of cellular response to phosphate starvation. Relationships: is a type of regulation of response to nutrient levels [GO:0032107]; is a type of regulation of cellular response to stress [GO:0080135]; regulates cellular response to phosphate starvation [GO:0016036]